{
  "gene_name": "Reticulon-1",
  "term_label": "postsynaptic density",
  "gene": "UniProtKB:Q16799",
  "term_id": "GO:0014069",
  "gene_symbol": "RTN1"
}